dUDP catabolic process [GO:0006257] (biological process) Relationships: is a type of pyrimidine deoxyribonucleoside diphosphate catabolic process [GO:0009198]; is a type of pyrimidine deoxyribonucleotide catabolic process [GO:0009223]; is a type of GO:0046077 Definition: The chemical reactions and pathways resulting in the breakdown of dUDP, deoxyuridine (5'-)diphosphate. Also known as: dUDP breakdown, dUDP catabolism, dUDP degradation Sources: ISBN:0198506732